{
  "gene_symbol": "AANAT",
  "term_id": "GO:0005737",
  "term_label": "cytoplasm",
  "gene_name": "Serotonin N-acetyltransferase",
  "gene": "UniProtKB:Q16613"
}